{
  "term_id": "UNKNOWN:0001",
  "gene_name": "Pleckstrin-2",
  "gene": "UniProtKB:Q9NYT0",
  "gene_symbol": "PLEK2",
  "term_label": "Unknown molecular function"
}